{
  "term_label": "DNA-binding transcription factor activity, RNA polymerase II-specific",
  "gene": "UniProtKB:Q8WYA1",
  "term_id": "GO:0000981",
  "gene_symbol": "BMAL2",
  "gene_name": "Basic helix-loop-helix ARNT-like protein 2"
}